{
  "gene_name": "MAP kinase-interacting serine_threonine-protein kinase 2",
  "gene_symbol": "MKNK2",
  "gene": "UniProtKB:Q9HBH9",
  "term_label": "calmodulin binding",
  "term_id": "GO:0005516"
}